{
  "gene": "UniProtKB:Q9H7X0",
  "gene_name": "N-alpha-acetyltransferase 60",
  "term_id": "GO:0004402",
  "gene_symbol": "NAA60",
  "term_label": "histone acetyltransferase activity"
}